positive regulation of heart rate by epinephrine-norepinephrine [GO:0001996] (biological process) Also known as: positive regulation of cardiac contraction rate by epinephrine-norepinephrine, positive regulation of heart contraction rate by adrenaline-noradrenaline, up regulation of heart contraction rate by epinephrine-norepinephrine, up-regulation of heart contraction rate by epinephrine-norepinephrine, upregulation of heart contraction rate by epinephrine-norepinephrine, activation of heart contraction rate by epinephrine-norepinephrine, stimulation of heart contraction rate by epinephrine-norepinephrine, increased chronotropy by epinephrine-norepinephrine, positive control of heart contraction rate by epinephrine-norepinephrine, positive regulation of heart contraction rate by epinephrine-norepinephrine Definition: The process in which the presence of epinephrine or norepinephrine in the bloodstream activates, maintains or increases the rate of heart contraction. Sources: GOC:dph Relationships: is a type of positive regulation of heart rate [GO:0010460]; is part of GO:0003321